RNA polymerase IV transcription repressor complex [GO:0090573] (cellular component) Sources: GOC:tb Relationships: is_a transcription repressor complex [GO:0017053]; is_a nuclear protein-containing complex [GO:0140513] Definition: A protein complex, located in the nucleus, that possesses activity that prevents or downregulates transcription from a RNA polymerase IV promoter.